{
  "gene_name": "Centrosome-associated protein ALMS1",
  "gene": "UniProtKB:Q8TCU4",
  "term_id": "GO:0005813",
  "gene_symbol": "ALMS1",
  "term_label": "centrosome"
}